{
  "gene_name": "Epithelial splicing regulatory protein 1",
  "term_id": "GO:0005654",
  "term_label": "nucleoplasm",
  "gene": "UniProtKB:Q6NXG1",
  "gene_symbol": "ESRP1"
}